{
  "gene": "UniProtKB:Q9Y5G6",
  "term_id": "GO:0005886",
  "gene_symbol": "PCDHGA7",
  "term_label": "plasma membrane",
  "gene_name": "Protocadherin gamma-A7"
}